{
  "term_label": "protein localization to plasma membrane",
  "gene_name": "Receptor activity-modifying protein 2",
  "gene_symbol": "RAMP2",
  "term_id": "GO:0072659",
  "gene": "UniProtKB:O60895"
}